pseudopodium assembly [GO:0031269] (biological process) Definition: The assembly of a pseudopodium by rearrangement of the actin cytoskeleton and overlying membrane. Regulation: regulated by GO:0031272; negatively regulated by GO:0031273; positively regulated by GO:0031274 Subtypes: extension of a leading process involved in cell motility in cerebral cortex radial glia guided migration [GO:0021816], lateral pseudopodium assembly [GO:0031271] Also known as: pseudopodium extension, pseudopodium formation Sources: GOC:dph, GOC:mah, GOC:pg, GOC:tb Relationships: is a type of pseudopodium organization [GO:0031268]; is a type of plasma membrane bounded cell projection assembly [GO:0120031]